gamma-secretase-Delta1 complex [GO:0070764] (cellular component) Relationships: is a type of GO:0098797 References: PMID:12794186 Definition: A protein complex that is formed by the association of the Notch ligand Delta1 with the gamma-secretase complex.